{
  "gene_symbol": "RGS18",
  "term_id": "GO:0009898",
  "gene_name": "Regulator of G-protein signaling 18",
  "term_label": "cytoplasmic side of plasma membrane",
  "gene": "UniProtKB:Q9NS28"
}